positive regulation of cyclase activity [GO:0031281] (biological process) Subtypes: positive regulation of guanylate cyclase activity [GO:0031284], positive regulation of adenylate cyclase activity [GO:0045762] Also known as: up regulation of cyclase activity, up-regulation of cyclase activity, upregulation of cyclase activity, activation of cyclase activity, stimulation of cyclase activity Definition: Any process that activates or increases the activity of a cyclase. Sources: GOC:mah Relationships: is a type of positive regulation of catalytic activity [GO:0043085]; positively regulates cyclase activity [GO:0009975]